{
  "gene": "UniProtKB:Q96GD3",
  "gene_symbol": "SCMH1",
  "term_label": "chromatin binding",
  "gene_name": "Polycomb protein SCMH1",
  "term_id": "GO:0003682"
}